cytosolic valyl-tRNA aminoacylation [GO:0061475] (biological process) Sources: GOC:dph Relationships: is a type of valyl-tRNA aminoacylation [GO:0006438]; occurs in cytosol [GO:0005829] Definition: The process of coupling valine to valyl-tRNA in the cytosol, catalyzed by valyl-tRNA synthetase. In tRNA aminoacylation, the amino acid is first activated by linkage to AMP and then transferred to either the 2'- or the 3'-hydroxyl group of the 3'-adenosine residue of the tRNA.